positive regulation of interleukin-2 production [GO:0032743] (biological process) Relationships: is a type of GO:0001819; is a type of regulation of interleukin-2 production [GO:0032663]; positively regulates interleukin-2 production [GO:0032623] Definition: Any process that activates or increases the frequency, rate, or extent of interleukin-2 production. Also known as: positive regulation of IL-2 production, up regulation of interleukin-2 production, up-regulation of interleukin-2 production, upregulation of interleukin-2 production, activation of interleukin-2 production, positive regulation of interleukin-2 biosynthetic process, positive regulation of interleukin-2 secretion, stimulation of interleukin-2 production Sources: GOC:mah